{
  "term_label": "synapse",
  "term_id": "GO:0045202",
  "gene": "UniProtKB:Q96S86",
  "gene_symbol": "HAPLN3",
  "gene_name": "Hyaluronan and proteoglycan link protein 3"
}